{
  "gene": "UniProtKB:P19256",
  "gene_name": "Lymphocyte function-associated antigen 3",
  "gene_symbol": "CD58",
  "term_label": "heterotypic cell-cell adhesion",
  "term_id": "GO:0034113"
}